response to environmental enrichment [GO:0090648] (biological process) Also known as: response to the introduction of novel objects Relationships: is a type of GO:0009605 References: PMID:23644055, PMID:25934034 Sources: GOC:sl Definition: Any process that results in a change in state or activity of an organism (in terms of movement, secretion, enzyme production, gene expression, etc.) as a result of the provision of a combination of complex inanimate and social stimulations in the organism's housing environment.